sphinganine-1-phosphate aldolase activity [GO:0008117] (MF) Sources: EC:4.1.2.27 Relationships: is a type of aldehyde-lyase activity [GO:0016832] Definition: Catalysis of the reaction: sphinganine 1-phosphate = phosphoethanolamine + palmitaldehyde. Also known as: dihydrosphingosine 1-phosphate aldolase activity, sphinganine-1-phosphate alkanal-lyase activity, sphinganine-1-phosphate lyase activity, sphinganine-1-phosphate palmitaldehyde-lyase (phosphoethanolamine-forming), sphinganine-1-phosphate palmitaldehyde-lyase activity, sphingosine-1-phosphate aldolase activity, sphingosine-1-phosphate lyase activity